negative regulation of mononuclear cell migration [GO:0071676] (biological process) Definition: Any process that decreases the rate, frequency or extent of mononuclear cell migration. Mononuclear cell migration is the movement of a mononuclear cell within or between different tissues and organs of the body. Subtypes: negative regulation of monocyte chemotaxis [GO:0090027], negative regulation of macrophage migration [GO:1905522], negative regulation of lymphocyte migration [GO:2000402], negative regulation of monocyte extravasation [GO:2000438], negative regulation of dendritic cell chemotaxis [GO:2000509] Sources: GOC:mah Also known as: down regulation of mononuclear cell migration, down-regulation of mononuclear cell migration, downregulation of mononuclear cell migration, inhibition of mononuclear cell migration Relationships: is a type of negative regulation of leukocyte migration [GO:0002686]; is_a regulation of mononuclear cell migration [GO:0071675]; negatively regulates mononuclear cell migration [GO:0071674]